maturation of LSU-rRNA [GO:0000470] (biological process) Relationships: is a type of rRNA processing [GO:0006364]; is part of ribosomal large subunit biogenesis [GO:0042273] Sources: GOC:curators Subtypes: GO:0000463, maturation of LSU-rRNA from tetracistronic rRNA transcript (SSU-rRNA, 5.8S rRNA, 2S rRNA, LSU-rRNA) [GO:0000473], GO:0000488, maturation of LSU-rRNA from tricistronic rRNA transcript (SSU-rRNA, LSU-rRNA,5S) [GO:0002108] Definition: Any process involved in the maturation of a precursor Large SubUnit (LSU) ribosomal RNA (rRNA) molecule into a mature LSU-rRNA molecule.